{
  "term_id": "GO:0000139",
  "gene_name": "Golgi apparatus membrane protein TVP23 homolog C",
  "term_label": "Golgi membrane",
  "gene": "UniProtKB:Q96ET8",
  "gene_symbol": "TVP23C"
}